{
  "term_id": "GO:0070175",
  "term_label": "positive regulation of enamel mineralization",
  "gene_symbol": "ENAM",
  "gene": "UniProtKB:Q9NRM1",
  "gene_name": "Enamelin"
}